{
  "term_id": "GO:0005829",
  "gene": "UniProtKB:Q96F44",
  "term_label": "cytosol",
  "gene_symbol": "TRIM11",
  "gene_name": "E3 ubiquitin-protein ligase TRIM11"
}